{
  "gene": "UniProtKB:O00459",
  "gene_symbol": "PIK3R2",
  "term_id": "GO:0008286",
  "gene_name": "Phosphatidylinositol 3-kinase regulatory subunit beta",
  "term_label": "insulin receptor signaling pathway"
}